tryptophanamidase activity [GO:0050365] (molecular function) Definition: Catalysis of the reaction: L-tryptophanamide + H2O = L-tryptophan + NH4. Relationships: is a type of hydrolase activity, acting on carbon-nitrogen (but not peptide) bonds, in linear amides [GO:0016811] Also known as: L-tryptophan aminopeptidase, tryptophan aminopeptidase, L-tryptophanamide amidohydrolase activity Sources: EC:3.5.1.57, RHEA:11012